{
  "term_label": "positive regulation of DNA-templated transcription",
  "gene": "UniProtKB:Q15650",
  "term_id": "GO:0045893",
  "gene_name": "Activating signal cointegrator 1",
  "gene_symbol": "TRIP4"
}